{
  "gene_name": "LON peptidase N-terminal domain and RING finger protein 2",
  "gene_symbol": "LONRF2",
  "term_label": "neuron projection development",
  "term_id": "GO:0031175",
  "gene": "UniProtKB:Q1L5Z9"
}